{
  "term_label": "Unknown cellular component",
  "gene_symbol": "PRR36",
  "gene_name": "Proline-rich protein 36",
  "gene": "UniProtKB:Q9H6K5",
  "term_id": "UNKNOWN:0003"
}